{
  "gene": "UniProtKB:P08133",
  "term_label": "calcium ion transport",
  "gene_symbol": "ANXA6",
  "gene_name": "Annexin A6",
  "term_id": "GO:0006816"
}